{
  "gene_name": "Zinc transporter ZIP11",
  "term_id": "GO:0071577",
  "gene_symbol": "SLC39A11",
  "term_label": "zinc ion transmembrane transport",
  "gene": "UniProtKB:Q8N1S5"
}